{
  "gene_symbol": "PNLIPRP3",
  "gene_name": "Pancreatic lipase-related protein 3",
  "gene": "UniProtKB:Q17RR3",
  "term_id": "GO:0004465",
  "term_label": "lipoprotein lipase activity"
}